{
  "gene": "UniProtKB:Q13573",
  "gene_symbol": "SNW1",
  "term_label": "Unknown molecular function",
  "term_id": "UNKNOWN:0001",
  "gene_name": "SNW domain-containing protein 1"
}